salutaridine synthase activity [GO:0047055] (molecular function) Definition: Catalysis of the reaction: (R)-reticuline + reduced [NADPH--hemoprotein reductase] + O2 = salutaridine + oxidized [NADPH--hemoprotein reductase] + 2 H2O + H+. Sources: RHEA:17713 Also known as: (R)-reticuline oxidase (C-C phenol-coupling) activity Relationships: is a type of oxidoreductase activity, acting on paired donors, with oxidation of a pair of donors resulting in the reduction of molecular oxygen to two molecules of water [GO:0016717]